{
  "gene_name": "Zinc finger protein 217",
  "gene_symbol": "ZNF217",
  "gene": "UniProtKB:O75362",
  "term_id": "GO:0005634",
  "term_label": "nucleus"
}